{
  "term_id": "GO:0005634",
  "gene": "UniProtKB:Q8N228",
  "term_label": "nucleus",
  "gene_symbol": "SCML4",
  "gene_name": "Sex comb on midleg-like protein 4"
}